{
  "gene_symbol": "KCNH7",
  "term_id": "GO:0071805",
  "term_label": "potassium ion transmembrane transport",
  "gene": "UniProtKB:Q9NS40",
  "gene_name": "Potassium voltage-gated channel subfamily H member 7"
}